{
  "gene_symbol": "PCDHGA1",
  "gene": "UniProtKB:Q9Y5H4",
  "term_label": "cell adhesion",
  "gene_name": "Protocadherin gamma-A1",
  "term_id": "GO:0007155"
}